L-ornithine transmembrane export from vacuole [GO:0089706] (biological process) Definition: The directed movement of L-ornithine out of the vacuole, across the vacuolar membrane. References: PMID:21307582 Relationships: is a type of GO:0032974; is a type of L-ornithine transmembrane transport [GO:1903352]